{
  "term_id": "GO:0005267",
  "term_label": "potassium channel activity",
  "gene": "UniProtKB:Q9NVV0",
  "gene_symbol": "TMEM38B",
  "gene_name": "Trimeric intracellular cation channel type B"
}